{
  "gene_symbol": "NDUFB1",
  "term_id": "UNKNOWN:0001",
  "gene_name": "NADH dehydrogenase [ubiquinone] 1 beta subcomplex subunit 1",
  "term_label": "Unknown molecular function",
  "gene": "UniProtKB:O75438"
}